hepatocyte growth factor receptor binding [GO:0005171] (molecular function) Relationships: is a type of GO:0070851 Sources: GOC:ai Definition: Binding to an hepatocyte growth factor receptor. Also known as: HGF receptor binding, hepatocyte growth factor, hepatocyte growth factor receptor ligand